{
  "gene_name": "NADH dehydrogenase [ubiquinone] 1 alpha subcomplex subunit 4-like 2",
  "gene": "UniProtKB:Q9NRX3",
  "term_id": "UNKNOWN:0002",
  "gene_symbol": "NDUFA4L2",
  "term_label": "Unknown biological process"
}